{
  "gene": "UniProtKB:O95400",
  "term_label": "Unknown biological process",
  "gene_symbol": "CD2BP2",
  "term_id": "UNKNOWN:0002",
  "gene_name": "CD2 antigen cytoplasmic tail-binding protein 2"
}